lignin biosynthetic process [GO:0009809] (biological process) Relationships: is a type of phenylpropanoid biosynthetic process [GO:0009699]; is a type of lignin metabolic process [GO:0009808] Sources: GOC:tair_curators, ISBN:0198547684 Definition: The chemical reactions and pathways resulting in the formation of lignins, a class of polymers formed by the dehydrogenetive radical polymerization of various phenylpropanoid monomers. Also known as: lignin anabolism, lignin biosynthesis, lignin formation, lignin synthesis Regulation: regulated by regulation of lignin biosynthetic process [GO:1901141] Subtypes: GO:1901060, guaiacyl lignin biosynthetic process [GO:1901063], syringal lignin biosynthetic process [GO:1901066]